{
  "term_label": "calcium-dependent phospholipid binding",
  "gene_name": "Annexin A7",
  "term_id": "GO:0005544",
  "gene": "UniProtKB:P20073",
  "gene_symbol": "ANXA7"
}